{
  "gene": "UniProtKB:Q16288",
  "gene_name": "NT-3 growth factor receptor",
  "term_id": "GO:0043121",
  "term_label": "neurotrophin binding",
  "gene_symbol": "NTRK3"
}